{
  "term_id": "GO:0044325",
  "gene_name": "TRPM8 channel-associated factor 1",
  "gene": "UniProtKB:Q9Y4C2",
  "term_label": "transmembrane transporter binding",
  "gene_symbol": "TCAF1"
}